alphav-beta3 integrin-PKCalpha complex [GO:0035866] (cellular component) Relationships: is a type of plasma membrane protein complex [GO:0098797] Definition: A protein complex that consists of an alphav-beta3 integrin complex bound to protein kinase C alpha. References: PMID:16014375 Sources: GOC:BHF, GOC:ebc Also known as: alphav-beta3 integrin-PKCa complex, alphav-beta3 integrin-protein kinase C alpha complex